{
  "term_label": "olfactory receptor activity",
  "gene_symbol": "OR10AG1",
  "term_id": "GO:0004984",
  "gene_name": "Olfactory receptor 10AG1",
  "gene": "UniProtKB:Q8NH19"
}